{
  "gene": "UniProtKB:A0A075B6Z5",
  "gene_symbol": "TRAJ4",
  "term_label": "Unknown molecular function",
  "gene_name": "T cell receptor alpha joining 4 (Fragment)",
  "term_id": "UNKNOWN:0001"
}